{
  "gene": "UniProtKB:O75908",
  "gene_symbol": "SOAT2",
  "term_id": "GO:0015485",
  "term_label": "cholesterol binding",
  "gene_name": "Sterol O-acyltransferase 2"
}